regulation of mitotic spindle elongation [GO:0032888] (biological process) Definition: Any process that modulates the frequency, rate or extent of the cell cycle process in which the distance is lengthened between poles of the mitotic spindle. Relationships: is a type of GO:0032887; is part of regulation of mitotic sister chromatid segregation [GO:0033047]; regulates mitotic spindle elongation [GO:0000022] Sources: GOC:mah Subtypes: regulation of mitotic spindle elongation (spindle phase three) [GO:0110162], negative regulation of mitotic spindle elongation [GO:1902845], positive regulation of mitotic spindle elongation [GO:1902846]